{
  "gene_symbol": "TACC3",
  "term_id": "GO:0005829",
  "gene_name": "Transforming acidic coiled-coil-containing protein 3",
  "gene": "UniProtKB:Q9Y6A5",
  "term_label": "cytosol"
}